{
  "term_label": "phospholipase activity",
  "gene_symbol": "ABHD16A",
  "term_id": "GO:0004620",
  "gene": "UniProtKB:O95870",
  "gene_name": "Phosphatidylserine lipase ABHD16A"
}